{
  "term_label": "calcium ion binding",
  "gene": "UniProtKB:P62760",
  "term_id": "GO:0005509",
  "gene_name": "Visinin-like protein 1",
  "gene_symbol": "VSNL1"
}